{
  "term_id": "UNKNOWN:0001",
  "gene": "UniProtKB:Q9P265",
  "gene_name": "Disco-interacting protein 2 homolog B",
  "gene_symbol": "DIP2B",
  "term_label": "Unknown molecular function"
}